regulation of torso signaling pathway [GO:0120175] (biological process) Definition: Any process that modulates the frequency, rate or extent of the torso signaling pathway. References: PMID:23732470 Sources: GOC:ha Relationships: is a type of regulation of signal transduction [GO:0009966]; regulates GO:0008293 Subtypes: positive regulation of torso signaling pathway [GO:0120176], GO:0120177